{
  "gene_name": "Basic leucine zipper transcriptional factor ATF-like",
  "term_id": "GO:0000981",
  "term_label": "DNA-binding transcription factor activity, RNA polymerase II-specific",
  "gene": "UniProtKB:Q16520",
  "gene_symbol": "BATF"
}